{
  "gene_name": "Telomeric repeat-binding factor 2-interacting protein 1",
  "gene": "UniProtKB:Q9NYB0",
  "gene_symbol": "TERF2IP",
  "term_label": "shelterin complex",
  "term_id": "GO:0070187"
}